{
  "gene": "UniProtKB:Q9BT78",
  "gene_name": "COP9 signalosome complex subunit 4",
  "term_label": "synaptic vesicle",
  "term_id": "GO:0008021",
  "gene_symbol": "COPS4"
}